hypoxanthine transport [GO:0035344] (BP) Definition: The directed movement of hypoxanthine, 6-hydroxypurine, into, out of or within a cell, or between cells, by means of some agent such as a transporter or pore. Sources: GOC:sl Also known as: 6-hydroxypurine transport, hypoxanthine transmembrane transport Relationships: is a type of purine nucleobase transport [GO:0006863] Regulation: regulated by GO:0035345; positively regulated by positive regulation of hypoxanthine transport [GO:0035346]; negatively regulated by negative regulation of hypoxanthine transport [GO:0035347]